{
  "term_label": "Unknown cellular component",
  "gene_symbol": "CINP",
  "gene": "UniProtKB:Q9BW66",
  "gene_name": "Cyclin-dependent kinase 2-interacting protein",
  "term_id": "UNKNOWN:0003"
}